negative regulation of haustorium mother cell formation [GO:0075195] (biological process) Note: Note that this term should not be used to annotate gene products of the host. It should only be used to annotate those gene products from the symbiont involved in this process. Definition: Any process that stops, prevents, or reduces the frequency, rate or extent of symbiont haustorium mother cell formation. The host is defined as the larger of the organisms involved in a symbiotic interaction. Relationships: is a type of negative regulation of developmental process [GO:0051093]; is a type of regulation of haustorium mother cell formation [GO:0075193]; negatively regulates haustorium mother cell formation [GO:0075192] Sources: GOC:pamgo_curators Also known as: negative regulation of haustorium mother cell formation on or near host